male germ-line cyst formation [GO:0048136] (biological process) References: PMID:10370240 Sources: GOC:jid Also known as: male germline cyst formation Relationships: is a type of germ-line cyst formation [GO:0048134]; is part of spermatogenesis [GO:0007283]; has part spermatogonial cell division [GO:0007284]; has part spermatocyte division [GO:0048137] Definition: Formation of a group of interconnected cells derived from a single male gonial founder cell.